{
  "gene_name": "Metalloproteinase inhibitor 2",
  "gene_symbol": "TIMP2",
  "term_label": "extracellular space",
  "term_id": "GO:0005615",
  "gene": "UniProtKB:P16035"
}